{
  "term_id": "GO:0003697",
  "gene": "UniProtKB:Q13156",
  "term_label": "single-stranded DNA binding",
  "gene_name": "Replication protein A 30 kDa subunit",
  "gene_symbol": "RPA4"
}